{
  "gene": "UniProtKB:P33681",
  "term_id": "GO:0006955",
  "gene_symbol": "CD80",
  "gene_name": "T-lymphocyte activation antigen CD80",
  "term_label": "immune response"
}